{
  "term_id": "GO:0005737",
  "term_label": "cytoplasm",
  "gene": "UniProtKB:P36405",
  "gene_name": "ADP-ribosylation factor-like protein 3",
  "gene_symbol": "ARL3"
}